{
  "gene_symbol": "NUMB",
  "term_label": "basolateral plasma membrane",
  "gene": "UniProtKB:P49757",
  "gene_name": "Protein numb homolog",
  "term_id": "GO:0016323"
}